{
  "gene": "UniProtKB:Q9P1Q0",
  "gene_name": "Vacuolar protein sorting-associated protein 54",
  "gene_symbol": "VPS54",
  "term_id": "GO:0042147",
  "term_label": "retrograde transport, endosome to Golgi"
}